{
  "gene_name": "tRNA-dihydrouridine(16_17) synthase [NAD(P)(+)]-like",
  "term_label": "tRNA dihydrouridine synthase activity",
  "gene_symbol": "DUS1L",
  "term_id": "GO:0017150",
  "gene": "UniProtKB:Q6P1R4"
}